DN4 thymocyte differentiation [GO:1904157] (BP) Definition: The process in which a relatively unspecialized cell acquires the specialized features of a DN4 thymocyte. A DN4 thymocyte is a CD4-,CD8- thymocyte that is also CD44-,CD25-. References: PMID:25398325 Sources: GOC:TermGenie, GOC:dph, GO_REF:0000086 Relationships: is a type of T cell differentiation in thymus [GO:0033077]